{
  "term_label": "microtubule",
  "gene": "UniProtKB:Q9BW30",
  "gene_name": "Tubulin polymerization-promoting protein family member 3",
  "term_id": "GO:0005874",
  "gene_symbol": "TPPP3"
}